pons structural organization [GO:0021585] (biological process) Sources: GOC:cls, GOC:dgh, GOC:dph, GOC:jid, GO_REF:0000021 Definition: The process that contributes to the act of creating the structural organization of the pons. This process pertains to the physical shaping of a rudimentary structure. The pons lies above the medulla and next to the cerebellum. The pons conveys information about movement from the cerebral hemisphere to the cerebellum. Also known as: pons structural organisation Relationships: is a type of anatomical structure arrangement [GO:0048532]; is part of hindbrain structural organization [GO:0021577]; is part of GO:0021583